{
  "gene_symbol": "SLAMF9",
  "gene": "UniProtKB:Q96A28",
  "term_label": "T cell activation",
  "gene_name": "SLAM family member 9",
  "term_id": "GO:0042110"
}